{
  "term_label": "regulation of DNA-templated transcription",
  "gene_symbol": "ZNF628",
  "term_id": "GO:0006355",
  "gene_name": "Zinc finger protein 628",
  "gene": "UniProtKB:Q5EBL2"
}